calcitonin family binding [GO:0097644] (molecular function) Definition: Binding to a member of the calcitonin family (e.g. adrenomedullin, adrenomedullin 2 (intermedin), amylin, calcitonin and calcitonin gene-related peptides (CGRPs)). Relationships: is a type of peptide hormone binding [GO:0017046] Subtypes: calcitonin binding [GO:0032841], amylin binding [GO:0097645], calcitonin gene-related peptide binding [GO:1990407], adrenomedullin binding [GO:1990409] References: PMID:10871296, PMID:12037140, PMID:18687416 Sources: GOC:bhm, InterPro:IPR021116